positive regulation of otic vesicle morphogenesis [GO:1904120] (BP) Also known as: up regulation of otic vesicle morphogenesis, up-regulation of otic vesicle morphogenesis, upregulation of otic vesicle morphogenesis, activation of otic vesicle morphogenesis Relationships: is_a GO:0110110; is a type of regulation of otic vesicle morphogenesis [GO:1904118]; is a type of positive regulation of morphogenesis of an epithelium [GO:1905332]; positively regulates otic vesicle morphogenesis [GO:0071600] Definition: Any process that activates or increases the frequency, rate or extent of otic vesicle morphogenesis. References: PMID:25677106 Sources: GOC:TermGenie, GO_REF:0000058